{
  "term_id": "GO:0016125",
  "gene_name": "UDP-glucuronosyltransferase 1A1",
  "term_label": "sterol metabolic process",
  "gene": "UniProtKB:P22309",
  "gene_symbol": "UGT1A1"
}